{
  "term_id": "UNKNOWN:0002",
  "gene_name": "Leucine-rich repeat and calponin homology domain-containing protein 4",
  "term_label": "Unknown biological process",
  "gene_symbol": "LRCH4",
  "gene": "UniProtKB:O75427"
}